regulation of amide metabolic process [GO:0034248] (biological process) Definition: Any process that modulates the frequency, rate or extent of the chemical reactions and pathways involving amides. Subtypes: regulation of penicillin catabolic process [GO:0033247], negative regulation of amide metabolic process [GO:0034249], positive regulation of amide metabolic process [GO:0034250], regulation of amide catabolic process [GO:0034251], GO:0043456, regulation of acyl-CoA biosynthetic process [GO:0050812], regulation of peptide hormone processing [GO:0060568], regulation of coenzyme A biosynthetic process [GO:0080020], regulation of penicillin biosynthetic process [GO:1900196], regulation of butyryl-CoA catabolic process to butanol [GO:1900497], regulation of butyryl-CoA catabolic process to butyrate [GO:1900500], regulation of emericellamide biosynthetic process [GO:1900658], regulation of gliotoxin biosynthetic process [GO:1900689], GO:1900707, GO:1900710, regulation of pseurotin A biosynthetic process [GO:1900849], GO:1901413, regulation of amyloid-beta formation [GO:1902003], regulation of glutathione biosynthetic process [GO:1903786], regulation of ferrichrome biosynthetic process [GO:1905568], regulation of ceramide biosynthetic process [GO:2000303], GO:2000752, regulation of sphingomyelin catabolic process [GO:2000754], regulation of isopentenyl diphosphate biosynthetic process, mevalonate pathway [GO:2001210] Also known as: regulation of amide metabolism, regulation of cellular amide metabolic process Relationships: is a type of regulation of metabolic process [GO:0019222]; regulates amide metabolic process [GO:0043603] Sources: GOC:mah